{
  "gene_name": "Disintegrin and metalloproteinase domain-containing protein 2",
  "gene_symbol": "ADAM2",
  "gene": "UniProtKB:Q99965",
  "term_id": "GO:0008584",
  "term_label": "male gonad development"
}